{
  "term_id": "UNKNOWN:0002",
  "gene_name": "Mortality factor 4-like protein 2",
  "term_label": "Unknown biological process",
  "gene_symbol": "MORF4L2",
  "gene": "UniProtKB:Q15014"
}